{
  "gene": "UniProtKB:Q96LB2",
  "gene_symbol": "MRGPRX1",
  "term_id": "GO:0007186",
  "gene_name": "Mas-related G-protein coupled receptor member X1",
  "term_label": "G protein-coupled receptor signaling pathway"
}